tRNA wobble adenosine to inosine editing [GO:0002100] (biological process) Relationships: is a type of tRNA wobble base modification [GO:0002097]; is a type of adenosine to inosine editing [GO:0006382] Sources: GOC:hjd, ISBN:155581073X Definition: The process in which an adenosine at position 34 of a tRNA is post-transcriptionally converted to inosine. The wobble nucleoside of the tRNA sequence  (position 34) corresponds to the first position of the anticodon.